{
  "gene_name": "DNA repair protein RAD51 homolog 1",
  "gene_symbol": "RAD51",
  "term_id": "GO:0008094",
  "gene": "UniProtKB:Q06609",
  "term_label": "ATP-dependent activity, acting on DNA"
}